clypeus morphogenesis [GO:0048721] (biological process) Relationships: is a type of post-embryonic animal morphogenesis [GO:0009886]; is part of clypeo-labral disc morphogenesis [GO:0007453]; is part of clypeus development [GO:0048723] Sources: GOC:rc Definition: The process in which the anatomical structures of the clypeus are generated and organized.